collagen type VII anchoring fibril [GO:0098652] (cellular component) Relationships: is a type of collagen anchoring fibril [GO:0098648] Definition: An antiparallel dimer of two collagen VII trimers, one end of which is embedded in the lamina densa while the other end attaches to banded collagen fibrils in the dermis. References: PMID:19693541